{
  "term_label": "mitochondrion",
  "gene_symbol": "MTRF1L",
  "term_id": "GO:0005739",
  "gene_name": "Peptide chain release factor 1-like, mitochondrial",
  "gene": "UniProtKB:Q9UGC7"
}